{
  "gene": "UniProtKB:Q9UN30",
  "term_label": "chromatin binding",
  "term_id": "GO:0003682",
  "gene_name": "Sex comb on midleg-like protein 1",
  "gene_symbol": "SCML1"
}